{
  "term_label": "extracellular space",
  "gene_name": "Peptidase inhibitor R3HDML",
  "gene_symbol": "R3HDML",
  "term_id": "GO:0005615",
  "gene": "UniProtKB:Q9H3Y0"
}